{
  "term_label": "protein kinase activity",
  "gene_symbol": "RIOK2",
  "term_id": "GO:0004672",
  "gene_name": "Serine_threonine-protein kinase RIO2",
  "gene": "UniProtKB:Q9BVS4"
}